mono-ADP-D-ribose binding [GO:0072571] (molecular function) References: PMID:20088964 Sources: GOC:mah, GOC:sart Also known as: mono-ADP-ribose binding, mADPr binding Definition: Binding to monomeric ADP-D-ribose, an ADP-aldose having ribose as the aldose fragment. Relationships: is a type of GO:0072570